{
  "gene_name": "Transcription factor Sp4",
  "term_id": "GO:0000981",
  "gene": "UniProtKB:Q02446",
  "term_label": "DNA-binding transcription factor activity, RNA polymerase II-specific",
  "gene_symbol": "SP4"
}